{
  "term_id": "GO:0055102",
  "term_label": "lipase inhibitor activity",
  "gene_symbol": "APOC3",
  "gene_name": "Apolipoprotein C-III",
  "gene": "UniProtKB:P02656"
}